{
  "term_id": "GO:0005886",
  "term_label": "plasma membrane",
  "gene_name": "Heme oxygenase 2",
  "gene_symbol": "HMOX2",
  "gene": "UniProtKB:P30519"
}